{
  "gene": "UniProtKB:P68363",
  "gene_symbol": "TUBA1B",
  "gene_name": "Tubulin alpha-1B chain",
  "term_id": "GO:0005200",
  "term_label": "structural constituent of cytoskeleton"
}